{
  "gene": "UniProtKB:Q9BUM1",
  "term_id": "GO:0016020",
  "gene_name": "Glucose-6-phosphatase 3",
  "term_label": "membrane",
  "gene_symbol": "G6PC3"
}